peptidyl-threonine autophosphorylation [GO:1990443] (biological process) References: PMID:7803855 Definition: The phosphorylation by a protein of one or more of its own threonine amino acid residues, or a threonine residue on an identical protein. Relationships: is a type of peptidyl-threonine phosphorylation [GO:0018107]; is a type of GO:0046777